saponin biosynthetic process [GO:0016135] (biological process) Relationships: is a type of saponin metabolic process [GO:0016134]; is a type of glycoside biosynthetic process [GO:0016138] Sources: GOC:go_curators Subtypes: GO:1904463 Also known as: saponin anabolism, saponin biosynthesis, saponin formation, saponin synthesis Definition: The chemical reactions and pathways resulting in the formation of saponins, glycosides of plants in which the aglycan (sapogenin) group is a terpene or steroid and the sugar group is a glucose, a galactose, a pentose, a methylpentose or an oligosaccharide. Saponins are powerful surfactant agents and membrane active; they are, hence, toxic to animals on injection.